secondary leaflet morphogenesis [GO:0060779] (biological process) Relationships: is a type of leaflet morphogenesis [GO:0060794] Sources: GOC:dph, GOC:sdb_2009, GOC:tb Definition: The process in which the secondary leaflet attains its shape. A secondary leaflet develops by branching or division of a primary leaflet.